{
  "term_id": "GO:0071539",
  "gene_symbol": "C2CD3",
  "gene": "UniProtKB:Q4AC94",
  "term_label": "protein localization to centrosome",
  "gene_name": "C2 domain-containing protein 3"
}